{
  "term_label": "DNA-binding transcription factor activity, RNA polymerase II-specific",
  "term_id": "GO:0000981",
  "gene_name": "Homeobox protein OTX2",
  "gene": "UniProtKB:P32243",
  "gene_symbol": "OTX2"
}